{
  "term_id": "GO:0007268",
  "gene_symbol": "CHRM2",
  "gene_name": "Muscarinic acetylcholine receptor M2",
  "term_label": "chemical synaptic transmission",
  "gene": "UniProtKB:P08172"
}